{
  "gene": "UniProtKB:Q99459",
  "gene_symbol": "CDC5L",
  "term_id": "GO:0000981",
  "gene_name": "Cell division cycle 5-like protein",
  "term_label": "DNA-binding transcription factor activity, RNA polymerase II-specific"
}